{
  "term_label": "Unknown biological process",
  "gene_name": "Transmembrane protein 9B",
  "term_id": "UNKNOWN:0002",
  "gene": "UniProtKB:Q9NQ34",
  "gene_symbol": "TMEM9B"
}